{
  "term_id": "GO:0005829",
  "gene_symbol": "USP17L15",
  "gene": "UniProtKB:C9J2P7",
  "gene_name": "Ubiquitin carboxyl-terminal hydrolase 17-like protein 15",
  "term_label": "cytosol"
}